{
  "gene": "UniProtKB:Q96PR1",
  "term_id": "GO:0032809",
  "gene_name": "Potassium voltage-gated channel subfamily C member 2",
  "term_label": "neuronal cell body membrane",
  "gene_symbol": "KCNC2"
}